longitudinal sarcoplasmic reticulum [GO:0014801] (cellular component) Sources: GOC:mtg_muscle Definition: The portion of the free sarcoplasmic reticulum consisting of longitudinal tubules that connect terminal cisternae. Relationships: is a type of GO:0110165; is part of sarcoplasmic reticulum [GO:0016529]